meiotic chromosome movement towards spindle pole [GO:0016344] (biological process) Relationships: is a type of GO:0051305; is a type of meiotic cell cycle process [GO:1903046]; is part of meiotic chromosome segregation [GO:0045132] Sources: GOC:ai Also known as: meiotic chromosome movement, chromosome migration to spindle pole during meiosis, chromosome movement towards spindle pole during meiosis, meiotic chromosome movement to spindle pole Subtypes: female meiotic chromosome movement towards spindle pole [GO:0016345], male meiotic chromosome movement towards spindle pole [GO:0016346], homologous chromosome movement towards spindle pole in meiosis I anaphase [GO:0051758], sister chromosome movement towards spindle pole involved in meiotic sister chromatid segregation [GO:0051759], meiotic centromere clustering [GO:1990571] Definition: The cell cycle process in which the directed movement of chromosomes from the center of the spindle towards the spindle poles takes place, mediated by the shortening of microtubules attached to the chromosomes. This occurs during meiosis.